{
  "term_id": "GO:0007165",
  "term_label": "signal transduction",
  "gene": "UniProtKB:Q9HBH0",
  "gene_symbol": "RHOF",
  "gene_name": "Rho-related GTP-binding protein RhoF"
}